regulation of pigment cell differentiation [GO:0050932] (biological process) Sources: GOC:ai Definition: Any process that modulates the frequency, rate or extent of pigmented cell differentiation. Subtypes: regulation of melanocyte differentiation [GO:0045634], regulation of leucophore differentiation [GO:0048775], regulation of erythrophore differentiation [GO:0048778], GO:0048781, regulation of iridophore differentiation [GO:0050937], regulation of xanthophore differentiation [GO:0050938], negative regulation of pigment cell differentiation [GO:0050941], GO:0050942 Relationships: is a type of regulation of cell differentiation [GO:0045595]; regulates pigment cell differentiation [GO:0050931]